{
  "gene_name": "Golgin subfamily A member 8N",
  "gene": "UniProtKB:F8WBI6",
  "term_label": "Golgi cisterna membrane",
  "gene_symbol": "GOLGA8N",
  "term_id": "GO:0032580"
}